{
  "term_id": "GO:0000981",
  "gene_name": "Krueppel-like factor 8",
  "gene_symbol": "KLF8",
  "term_label": "DNA-binding transcription factor activity, RNA polymerase II-specific",
  "gene": "UniProtKB:O95600"
}